{
  "gene_name": "Zinc finger protein PLAGL1",
  "term_id": "GO:0000978",
  "term_label": "RNA polymerase II cis-regulatory region sequence-specific DNA binding",
  "gene_symbol": "PLAGL1",
  "gene": "UniProtKB:Q9UM63"
}